{
  "gene_symbol": "JAK1",
  "term_label": "growth hormone receptor binding",
  "term_id": "GO:0005131",
  "gene_name": "Tyrosine-protein kinase JAK1",
  "gene": "UniProtKB:P23458"
}